{
  "gene_symbol": "IFNAR1",
  "term_id": "GO:0004905",
  "gene": "UniProtKB:P17181",
  "term_label": "type I interferon receptor activity",
  "gene_name": "Interferon alpha_beta receptor 1"
}